{
  "gene_name": "Microtubule-associated serine_threonine-protein kinase 1",
  "term_label": "neuronal cell body",
  "term_id": "GO:0043025",
  "gene_symbol": "MAST1",
  "gene": "UniProtKB:Q9Y2H9"
}